glyoxal metabolic process [GO:1903189] (biological process) Relationships: is a type of aldehyde metabolic process [GO:0006081] Definition: The chemical reactions and pathways involving glyoxal. Subtypes: protein deglycation, glyoxal removal [GO:0036529], GO:1903190, glyoxal biosynthetic process [GO:1903191] Sources: GOC:PARL, GOC:TermGenie, GOC:bf, GO_REF:0000068 Also known as: glyoxal metabolism